{
  "gene_symbol": "IL5RA",
  "gene_name": "Interleukin-5 receptor subunit alpha",
  "term_id": "GO:0004896",
  "term_label": "cytokine receptor activity",
  "gene": "UniProtKB:Q01344"
}